{
  "term_id": "UNKNOWN:0003",
  "gene": "UniProtKB:A6NEH8",
  "gene_symbol": "ZNF503-AS2",
  "term_label": "Unknown cellular component",
  "gene_name": "Putative uncharacterized protein encoded by ZNF503-AS2"
}